{
  "term_label": "Unknown molecular function",
  "gene_symbol": "TBCC",
  "term_id": "UNKNOWN:0001",
  "gene": "UniProtKB:Q15814",
  "gene_name": "Tubulin-specific chaperone C"
}